{
  "term_id": "GO:0035556",
  "gene": "UniProtKB:Q96L50",
  "gene_name": "Leucine-rich repeat protein 1",
  "term_label": "intracellular signal transduction",
  "gene_symbol": "LRR1"
}